protein localization to medial cortex [GO:0071574] (biological process) Also known as: protein localisation to medial cortex Regulation: regulated by regulation of protein localization to medial cortex [GO:0106011]; positively regulated by positive regulation of protein localization to medial cortex [GO:0106012]; negatively regulated by negative regulation of protein localization to medial cortex [GO:0140325] Definition: A process in which a protein is transported to, or maintained in, the medial cortex. Sources: GOC:mah Subtypes: protein localization to medial cortical node [GO:1902577] Relationships: is a type of protein localization to cell cortex [GO:0072697]; is a type of protein localization to cell division site [GO:0072741]